ribonuclease III complex [GO:1903095] (cellular component) Subtypes: microprocessor complex [GO:0070877] Definition: A protein complex which is capable of ribonuclease III activity. Relationships: is a type of endoribonuclease complex [GO:1902555] References: PMID:22393237 Sources: GOC:TermGenie, GOC:bhm, GO_REF:0000088 Note: An example of this is RNC in human (Q9NRR4) in PMID:22393237 (inferred from direct assay).